{
  "gene_symbol": "ASL",
  "term_id": "GO:0004056",
  "term_label": "argininosuccinate lyase activity",
  "gene_name": "Argininosuccinate lyase",
  "gene": "UniProtKB:P04424"
}